protein localization to bud neck [GO:0097271] (BP) Definition: A process in which a protein is transported to, or maintained at, a location within a cellular bud neck. Relationships: is a type of intracellular protein localization [GO:0008104] References: PMID:22344253 Sources: GOC:rb Also known as: protein localisation to bud neck, protein localization to cellular bud neck